{
  "gene": "UniProtKB:Q8IUI8",
  "gene_symbol": "CRLF3",
  "term_label": "DNA binding",
  "term_id": "GO:0003677",
  "gene_name": "Cytokine receptor-like factor 3"
}